{
  "gene_symbol": "CHMP6",
  "gene": "UniProtKB:Q96FZ7",
  "term_id": "GO:0005771",
  "term_label": "multivesicular body",
  "gene_name": "Charged multivesicular body protein 6"
}